{
  "gene": "UniProtKB:Q15365",
  "gene_symbol": "PCBP1",
  "gene_name": "Poly(rC)-binding protein 1",
  "term_label": "mRNA binding",
  "term_id": "GO:0003729"
}